{
  "gene_name": "Polyserase-2",
  "gene": "UniProtKB:Q5K4E3",
  "gene_symbol": "PRSS36",
  "term_label": "Unknown biological process",
  "term_id": "UNKNOWN:0002"
}